{
  "term_label": "plasma membrane",
  "gene": "UniProtKB:Q9H756",
  "gene_symbol": "LRRC19",
  "term_id": "GO:0005886",
  "gene_name": "Leucine-rich repeat-containing protein 19"
}